mesenchymal cell proliferation involved in ureter development [GO:0072198] (biological process) Regulation: regulated by regulation of mesenchymal cell proliferation involved in ureter development [GO:0072199]; negatively regulated by negative regulation of mesenchymal cell proliferation involved in ureter development [GO:0072200]; RO_0002213 by GO:2000729 Also known as: ureter mesenchymal cell proliferation, ureteral mesenchymal cell proliferation Definition: The multiplication or reproduction of cells, resulting in the expansion of a mesenchymal cell population of the ureter, that contributes to ureter development. Relationships: is a type of mesenchymal cell proliferation [GO:0010463]; is part of ureter development [GO:0072189] Sources: GOC:mtg_kidney_jan10